{
  "gene": "UniProtKB:Q12756",
  "gene_symbol": "KIF1A",
  "gene_name": "Kinesin-like protein KIF1A",
  "term_label": "ATP hydrolysis activity",
  "term_id": "GO:0016887"
}